{
  "gene_symbol": "ANK3",
  "gene": "UniProtKB:Q12955",
  "gene_name": "Ankyrin-3",
  "term_label": "spectrin binding",
  "term_id": "GO:0030507"
}